membraneless organelle assembly [GO:0140694] (biological process) Definition: The aggregation, arrangement and bonding together of a set of components to form a non-membrane-bounded organelle. Also known as: non-membrane-bounded organelle assembly, non-membrane-bounded organelle formation, non-membrane-enclosed organelle assembly, non-membrane-enclosed organelle formation References: PMID:28225081 Relationships: is a type of organelle assembly [GO:0070925] Subtypes: septin ring assembly [GO:0000921], myofibril assembly [GO:0030239], P-body assembly [GO:0033962], GO:0034063, ribosome assembly [GO:0042255], cellulosome assembly [GO:0044575], bacterial-type flagellum assembly [GO:0044780], spindle assembly [GO:0051225], kinetochore assembly [GO:0051382], podosome assembly [GO:0071800], GO:0098534, GO:0140042, GO:0140167, terminal web assembly [GO:1902896], proteasome storage granule assembly [GO:1902906], P granule assembly [GO:1903863], GO:1904258, cytoplasmic U snRNP body assembly [GO:1990194]